{
  "gene_symbol": "Q6ZQT0",
  "term_label": "Unknown cellular component",
  "gene": "UniProtKB:Q6ZQT0",
  "gene_name": "Putative uncharacterized protein FLJ45035",
  "term_id": "UNKNOWN:0003"
}